{
  "gene_symbol": "TRMT13",
  "gene_name": "tRNA:m(4)X modification enzyme TRM13 homolog",
  "term_id": "GO:0008175",
  "term_label": "tRNA methyltransferase activity",
  "gene": "UniProtKB:Q9NUP7"
}